homocarnosine synthase activity [GO:0102102] (molecular function) Relationships: is a type of acid-amino acid ligase activity [GO:0016881] Sources: GOC:pz Definition: Catalysis of the reaction: gamma-aminobutyric acid + L-histidine + ATP = H+ + homocarnosine + ADP + hydrogenphosphate.